basophil mediated immunity [GO:0002560] (biological process) Subtypes: type I hypersensitivity mediated by basophils [GO:0002559] Sources: GOC:add, ISBN:0781735149 Definition: Any process involved in the carrying out of an immune response by a basophil. Relationships: is a type of myeloid leukocyte mediated immunity [GO:0002444]